{
  "term_label": "'de novo' cotranslational protein folding",
  "gene_symbol": "DNAJC2",
  "term_id": "GO:0051083",
  "gene_name": "DnaJ homolog subfamily C member 2",
  "gene": "UniProtKB:Q99543"
}